{
  "gene_name": "Protocadherin alpha-C1",
  "term_label": "plasma membrane",
  "term_id": "GO:0005886",
  "gene": "UniProtKB:Q9H158",
  "gene_symbol": "PCDHAC1"
}